cyanide metabolic process [GO:0019499] (biological process) Relationships: is a type of GO:0008152 Also known as: cyanide metabolism Subtypes: GO:0019500, GO:0046202 Definition: The chemical reactions and pathways involving cyanide, NC-, the anion of hydrocyanic acid. Cyanide is a potent inhibitor of respiration, reacting with the ferric form of cytochrome aa3 and thus blocking the electron transport chain. Sources: ISBN:0198506732